{
  "term_label": "chemotaxis",
  "term_id": "GO:0006935",
  "gene_name": "Eosinophil cationic protein",
  "gene_symbol": "RNASE3",
  "gene": "UniProtKB:P12724"
}